{
  "term_label": "Unknown biological process",
  "term_id": "UNKNOWN:0002",
  "gene_name": "T cell receptor alpha joining 35 (non-functional) (Fragment)",
  "gene_symbol": "TRAJ35",
  "gene": "UniProtKB:A0A075B6Y2"
}